blood vessel endothelial cell proliferation involved in sprouting angiogenesis [GO:0002043] (biological process) Relationships: is a type of endothelial cell proliferation [GO:0001935]; is part of sprouting angiogenesis [GO:0002040] References: PMID:16391003 Sources: GOC:dph, GOC:tb Regulation: regulated by regulation of blood vessel endothelial cell proliferation involved in sprouting angiogenesis [GO:1903587]; negatively regulated by negative regulation of blood vessel endothelial cell proliferation involved in sprouting angiogenesis [GO:1903588]; positively regulated by positive regulation of blood vessel endothelial cell proliferation involved in sprouting angiogenesis [GO:1903589] Definition: The multiplication or reproduction of blood vessel endothelial cells, resulting in the expansion of a cell population contributing to sprouting angiogenesis. Also known as: blood vessel endothelial cell proliferation during sprouting angiogenesis